{
  "term_label": "positive regulation of ERK1 and ERK2 cascade",
  "term_id": "GO:0070374",
  "gene_symbol": "ARRB2",
  "gene": "UniProtKB:P32121",
  "gene_name": "Beta-arrestin-2"
}